{
  "gene_name": "Equilibrative nucleoside transporter 2",
  "term_label": "thymine transport",
  "term_id": "GO:0035364",
  "gene_symbol": "SLC29A2",
  "gene": "UniProtKB:Q14542"
}